{
  "gene_symbol": "KRTAP5-9",
  "term_label": "Unknown molecular function",
  "gene_name": "Keratin-associated protein 5-9",
  "gene": "UniProtKB:P26371",
  "term_id": "UNKNOWN:0001"
}